{
  "gene_name": "NEDD8-conjugating enzyme UBE2F",
  "term_label": "nucleus",
  "gene_symbol": "UBE2F",
  "term_id": "GO:0005634",
  "gene": "UniProtKB:Q969M7"
}